response to ATP [GO:0033198] (biological process) Relationships: is a type of response to purine-containing compound [GO:0014074]; is a type of response to organophosphorus [GO:0046683]; is a type of GO:1901700 Also known as: response to adenosine 5'-triphosphate, response to adenosine triphosphate Subtypes: cellular response to ATP [GO:0071318] Sources: GOC:sl Definition: Any process that results in a change in state or activity of a cell or an organism (in terms of movement, secretion, enzyme production, gene expression, etc.) as a result of an ATP (adenosine 5'-triphosphate) stimulus.